{
  "term_label": "cis-Golgi network",
  "gene": "UniProtKB:Q99996",
  "term_id": "GO:0005801",
  "gene_name": "A-kinase anchor protein 9",
  "gene_symbol": "AKAP9"
}